{
  "gene_symbol": "ATOH7",
  "gene_name": "Transcription factor ATOH7",
  "term_id": "GO:0045944",
  "gene": "UniProtKB:Q8N100",
  "term_label": "positive regulation of transcription by RNA polymerase II"
}